{
  "gene_symbol": "RPS2",
  "gene": "UniProtKB:P15880",
  "term_label": "structural constituent of ribosome",
  "term_id": "GO:0003735",
  "gene_name": "Small ribosomal subunit protein uS5"
}